response to chondroitin 4'-sulfate [GO:1905441] (biological process) Definition: Any process that results in a change in state or activity of a cell or an organism (in terms of movement, secretion, enzyme production, gene expression, etc.) as a result of a chondroitin 4'-sulfate stimulus. References: PMID:22365850 Sources: GOC:TermGenie, GO_REF:0000071 Relationships: is_a response to nitrogen compound [GO:1901698]; is a type of response to oxygen-containing compound [GO:1901700] Subtypes: cellular response to chondroitin 4'-sulfate [GO:1905442]